8-oxo-7,8-dihydrodeoxyguanosine triphosphate pyrophosphatase activity [GO:0035539] (molecular function) References: PMID:17804481, PMID:7782328, PMID:7859359 Sources: RHEA:31575 Relationships: is a type of GO:0047429 Also known as: 8-oxo-7,8-dihydro-2'-deoxyguanosine 5'-triphosphate pyrophosphohydrolase activity, 8-oxo-7,8-dihydro-deoxyguanosine triphosphate pyrophosphatase activity, 8-oxo-7,8-dihydrodeoxyguanosine triphosphatase activity, 8-oxo-dGTP pyrophosphohydrolase activity, 8-oxo-dGTPase activity Definition: Catalysis of the reaction: 8-oxo-7,8-dihydrodeoxyguanosine-triphosphate (8-oxo-dGTP) + H2O = 8-oxo-7,8-dihydrodeoxyguanosine phosphate (8-oxo-dGMP) + diphosphate. 8-oxo-dGTP is the oxidised form of the free guanine nucleotide and can act as a potent mutagenic substrate for DNA synthesis causing transversion mutations. 8-oxo-dGTPase hydrolyses 8-oxo-dGTP to its monophosphate form to prevent the misincorporation of 8-oxo-dGTP into cellular DNA.